{
  "term_label": "anterior/posterior pattern specification",
  "term_id": "GO:0009952",
  "gene_name": "Homeobox protein Hox-B7",
  "gene_symbol": "HOXB7",
  "gene": "UniProtKB:P09629"
}